chromosome organization [GO:0051276] (biological process) Also known as: DNA condensation, chromosome organisation, DNA packaging, chromosome organization and biogenesis, maintenance of genome integrity, nuclear genome maintenance Regulation: regulated by GO:0033044; negatively regulated by GO:2001251; positively regulated by positive regulation of chromosome organization [GO:2001252] Definition: A process that is carried out at the cellular level that results in the assembly, arrangement of constituent parts, or disassembly of chromosomes, structures composed of a very long molecule of DNA and associated proteins that carries hereditary information. This term covers covalent modifications at the molecular level as well as spatial relationships among the major components of a chromosome. Sources: GOC:ai, GOC:dph, GOC:jl, GOC:mah Subtypes: nucleotide-excision repair, DNA damage recognition [GO:0000715], sister chromatid segregation [GO:0000819], transcription-dependent tethering of RNA polymerase II gene DNA at nuclear periphery [GO:0000972], sister chromatid cohesion [GO:0007062], GO:0030261, telomere organization [GO:0032200], polytene chromosome puffing [GO:0035079], bacterial nucleoid DNA packaging [GO:0036386], maintenance of DNA repeat elements [GO:0043570], kinetochore organization [GO:0051383], tRNA gene clustering [GO:0070058], GO:0070192, synaptonemal complex organization [GO:0070193], DNA conformation change [GO:0071103], GO:0090139, GO:0141112, plastid chromosome packaging [GO:1900160] Relationships: is a type of GO:0006996